regulation of late endosome to lysosome transport [GO:1902822] (biological process) Subtypes: negative regulation of late endosome to lysosome transport [GO:1902823], positive regulation of late endosome to lysosome transport [GO:1902824] Relationships: is_a regulation of vacuolar transport [GO:1903335]; regulates GO:1902774 Definition: Any process that modulates the frequency, rate or extent of late endosome to lysosome transport. References: PMID:23949442 Sources: GOC:PARL, GOC:TermGenie, GOC:pad, GO_REF:0000058 Also known as: regulation of prevacuolar compartment to lysosome transport